{
  "gene": "UniProtKB:Q8NEY8",
  "term_id": "GO:0045814",
  "term_label": "negative regulation of gene expression, epigenetic",
  "gene_symbol": "PPHLN1",
  "gene_name": "Periphilin-1"
}